{
  "term_id": "GO:0000977",
  "term_label": "RNA polymerase II transcription regulatory region sequence-specific DNA binding",
  "gene_name": "Homeobox protein CDX-2",
  "gene": "UniProtKB:Q99626",
  "gene_symbol": "CDX2"
}